{
  "term_id": "GO:0005768",
  "gene_name": "Thymus-specific serine protease",
  "gene": "UniProtKB:Q9NQE7",
  "term_label": "endosome",
  "gene_symbol": "PRSS16"
}